{
  "gene_name": "LIM domain kinase 2",
  "gene": "UniProtKB:P53671",
  "term_label": "protein serine/threonine kinase activity",
  "term_id": "GO:0004674",
  "gene_symbol": "LIMK2"
}